{
  "term_label": "cytoplasm",
  "term_id": "GO:0005737",
  "gene": "UniProtKB:Q9UQC2",
  "gene_symbol": "GAB2",
  "gene_name": "GRB2-associated-binding protein 2"
}